{
  "gene": "UniProtKB:P15056",
  "term_id": "GO:0005829",
  "gene_name": "Serine_threonine-protein kinase B-raf",
  "term_label": "cytosol",
  "gene_symbol": "BRAF"
}